{
  "gene_symbol": "TBX1",
  "term_id": "GO:0000785",
  "gene": "UniProtKB:O43435",
  "term_label": "chromatin",
  "gene_name": "T-box transcription factor TBX1"
}